secondary shoot formation [GO:0010223] (biological process) Definition: The process that gives rise to secondary (or auxiliary or axillary) shoots in plants. This process pertains to the initial formation of a structure from unspecified parts. These secondary shoots originate from secondary meristems initiated in the axils of leaf primordia. Axillary meristems function like the shoot apical meristem of the primary shoot initiating the development of lateral organs. References: PMID:12815068 Sources: GOC:tb Relationships: is a type of morphogenesis of a branching structure [GO:0001763]; is a type of shoot axis formation [GO:0010346] Regulation: regulated by regulation of secondary shoot formation [GO:2000032] Also known as: axillary shoot system formation, auxiliary shoot formation, axillary shoot formation, shoot branching